box C/D sno(s)RNA 3'-end processing [GO:0000494] (biological process) Relationships: is a type of sno(s)RNA 3'-end processing [GO:0031126]; is a type of box C/D sno(s)RNA processing [GO:0034963] Sources: GOC:krc Definition: Any process involved in forming the mature 3' end of a box C/D RNA molecule. Also known as: box C/D RNA 3' end processing, box C/D sRNA 3'-end processing, box C/D snoRNA 3'-end processing